positive regulation of toll-like receptor signaling pathway [GO:0034123] (biological process) References: PMID:16551253, PMID:17328678 Sources: GOC:add Relationships: is a type of regulation of toll-like receptor signaling pathway [GO:0034121]; is a type of positive regulation of pattern recognition receptor signaling pathway [GO:0062208]; positively regulates toll-like receptor signaling pathway [GO:0002224] Also known as: positive regulation of TLR signaling pathway, positive regulation of toll-like receptor signalling pathway Definition: Any process that activates or increases the frequency, rate, or extent of toll-like receptor signaling pathway. Subtypes: positive regulation of MyD88-dependent toll-like receptor signaling pathway [GO:0034126], positive regulation of MyD88-independent toll-like receptor signaling pathway [GO:0034129], positive regulation of toll-like receptor 21 signaling pathway [GO:2000445]